{
  "gene_name": "DNA topoisomerase 2-binding protein 1",
  "term_id": "GO:0033314",
  "gene": "UniProtKB:Q92547",
  "gene_symbol": "TOPBP1",
  "term_label": "mitotic DNA replication checkpoint signaling"
}